{
  "term_label": "Unknown biological process",
  "gene_name": "cAMP-regulated phosphoprotein 19",
  "gene_symbol": "ARPP19",
  "term_id": "UNKNOWN:0002",
  "gene": "UniProtKB:P56211"
}